{
  "term_id": "GO:0043195",
  "term_label": "terminal bouton",
  "gene_name": "Alpha-soluble NSF attachment protein",
  "gene": "UniProtKB:P54920",
  "gene_symbol": "NAPA"
}